negative regulation of natural killer cell activation [GO:0032815] (biological process) Relationships: is a type of GO:0032814; is a type of negative regulation of lymphocyte activation [GO:0051250]; negatively regulates GO:0030101 Definition: Any process that stops, prevents, or reduces the frequency, rate or extent of natural killer cell activation. Sources: GOC:mah Also known as: down regulation of natural killer cell activation, down-regulation of natural killer cell activation, downregulation of natural killer cell activation, negative regulation of NK cell activation, inhibition of natural killer cell activation Subtypes: negative regulation of natural killer cell proliferation [GO:0032818], negative regulation of natural killer cell differentiation [GO:0032824]